{
  "term_label": "Unknown molecular function",
  "gene_name": "Putative uncharacterized protein encoded by LINC00167",
  "term_id": "UNKNOWN:0001",
  "gene_symbol": "PRDM10-DT",
  "gene": "UniProtKB:Q96N53"
}